{
  "gene_symbol": "KLRG1",
  "gene_name": "Killer cell lectin-like receptor subfamily G member 1",
  "term_label": "Unknown biological process",
  "term_id": "UNKNOWN:0002",
  "gene": "UniProtKB:Q96E93"
}